{
  "gene_symbol": "ZNF35",
  "gene": "UniProtKB:P13682",
  "term_id": "GO:0000977",
  "term_label": "RNA polymerase II transcription regulatory region sequence-specific DNA binding",
  "gene_name": "Zinc finger protein 35"
}